{
  "term_label": "negative regulation of transcription by RNA polymerase II",
  "gene_symbol": "BCOR",
  "term_id": "GO:0000122",
  "gene": "UniProtKB:Q6W2J9",
  "gene_name": "BCL-6 corepressor"
}